actin filament bundle [GO:0032432] (CC) Also known as: actin cable Relationships: is a type of cellular anatomical structure [GO:0110165]; is part of GO:0015629; has part actin filament [GO:0005884] Subtypes: actin rod [GO:0031002], GO:0031003, contractile actin filament bundle [GO:0097517], parallel actin filament bundle [GO:0097518] Definition: An assembly of actin filaments that are on the same axis but may be oriented with the same or opposite polarities and may be packed with different levels of tightness. Sources: GOC:mah